{
  "term_label": "RNA polymerase II cis-regulatory region sequence-specific DNA binding",
  "term_id": "GO:0000978",
  "gene_symbol": "VDR",
  "gene_name": "Vitamin D3 receptor",
  "gene": "UniProtKB:P11473"
}